{
  "gene": "UniProtKB:A0A1B0GTR3",
  "term_label": "Unknown molecular function",
  "gene_name": "Uncharacterized protein CXorf51A",
  "term_id": "UNKNOWN:0001",
  "gene_symbol": "CXorf51A"
}